{
  "gene": "UniProtKB:Q9UKF5",
  "term_id": "GO:0009897",
  "term_label": "external side of plasma membrane",
  "gene_symbol": "ADAM29",
  "gene_name": "Disintegrin and metalloproteinase domain-containing protein 29"
}